{
  "term_id": "UNKNOWN:0001",
  "gene_name": "Reticulophagy regulator 3",
  "term_label": "Unknown molecular function",
  "gene": "UniProtKB:Q86VR2",
  "gene_symbol": "RETREG3"
}